T=1 icosahedral viral capsid [GO:0039615] (cellular component) Definition: The protein coat that surrounds the infective nucleic acid in some virus particles where the subunits (capsomeres) are arranged to form an icosahedron with T=1 symmetry. The T=1 capsid is composed of 12 pentameric capsomeres. Sources: VZ:1057 Relationships: is a type of GO:0019030